sphingosine-1-phosphate receptor activity [GO:0038036] (molecular function) Definition: Combining with the sphingolipid sphingosine-1-phosphate (S1P), and transmitting the signal across the membrane by activating an associated G-protein. Also known as: S1P receptor activity Relationships: is a type of bioactive lipid receptor activity [GO:0045125]; is part of sphingosine-1-phosphate receptor signaling pathway [GO:0003376] References: PMID:12728273 Sources: GOC:bf, Wikipedia:S1PR1